{
  "term_id": "GO:0008146",
  "gene": "UniProtKB:Q6IMI4",
  "gene_name": "Sulfotransferase 6B1",
  "term_label": "sulfotransferase activity",
  "gene_symbol": "SULT6B1"
}